{
  "gene": "UniProtKB:Q8NBK3",
  "term_label": "endoplasmic reticulum",
  "gene_symbol": "SUMF1",
  "term_id": "GO:0005783",
  "gene_name": "Formylglycine-generating enzyme"
}